2,6-beta-fructan 6-levanbiohydrolase activity [GO:0033912] (molecular function) Sources: EC:3.2.1.64 Relationships: is a type of GO:0004553 Definition: Catalysis of the hydrolysis of (2->6)-beta-D-fructofuranan, to remove successive disaccharide residues as levanbiose, i.e. 6-(beta-D-fructofuranosyl)-D-fructose, from the end of the chain. Also known as: 2,6-beta-D-fructan 6-beta-D-fructofuranosylfructohydrolase activity, 2,6-beta-D-fructan 6-levanbiohydrolase activity, 2,6-beta-D-fructofuranan 6-(beta-D-fructosyl)-D-fructose-hydrolase activity, beta-2,6-fructan-6-levanbiohydrolase activity, levanbiose-producing levanase activity